{
  "term_label": "nucleus",
  "gene": "UniProtKB:Q52M93",
  "gene_name": "Zinc finger protein 585B",
  "term_id": "GO:0005634",
  "gene_symbol": "ZNF585B"
}